basal dendrite arborization [GO:0150020] (biological process) Definition: The process in which the anatomical structures of a dendritic tree are generated on the basal neuron side and organized into dendritic branches. Relationships: is a type of dendrite arborization [GO:0140059]; is a type of GO:0150019 References: PMID:22683681 Sources: GOC:aruk, GOC:bc